{
  "term_id": "GO:0000981",
  "gene_symbol": "ZNF486",
  "term_label": "DNA-binding transcription factor activity, RNA polymerase II-specific",
  "gene_name": "Zinc finger protein 486",
  "gene": "UniProtKB:Q96H40"
}